{
  "gene_name": "AP-4 complex subunit epsilon-1",
  "gene": "UniProtKB:Q9UPM8",
  "gene_symbol": "AP4E1",
  "term_id": "GO:0030124",
  "term_label": "AP-4 adaptor complex"
}